{
  "gene_name": "CCR4-NOT transcription complex subunit 9",
  "gene": "UniProtKB:Q92600",
  "gene_symbol": "CNOT9",
  "term_id": "GO:0017148",
  "term_label": "negative regulation of translation"
}